{
  "gene": "UniProtKB:Q9UJT0",
  "gene_symbol": "TUBE1",
  "term_label": "structural constituent of cytoskeleton",
  "term_id": "GO:0005200",
  "gene_name": "Tubulin epsilon chain"
}